negative regulation of cell adhesion [GO:0007162] (biological process) Sources: GOC:go_curators Subtypes: GO:0006933, GO:0010812, GO:0021804, GO:0022408, negative regulation of cell adhesion mediated by integrin [GO:0033629], negative regulation of cell adhesion involved in sprouting angiogenesis [GO:0106089] Relationships: is a type of regulation of cell adhesion [GO:0030155]; is a type of negative regulation of cellular process [GO:0048523]; negatively regulates GO:0007155 Also known as: down regulation of cell adhesion, down-regulation of cell adhesion, downregulation of cell adhesion, inhibition of cell adhesion, cell adhesion receptor inhibitor activity Definition: Any process that stops, prevents, or reduces the frequency, rate or extent of cell adhesion.